{
  "term_label": "cytoplasm",
  "gene_name": "PAS domain-containing serine_threonine-protein kinase",
  "gene": "UniProtKB:Q96RG2",
  "gene_symbol": "PASK",
  "term_id": "GO:0005737"
}